{
  "gene_name": "rRNA 2'-O-methyltransferase fibrillarin",
  "gene_symbol": "FBL",
  "gene": "UniProtKB:P22087",
  "term_id": "GO:0000494",
  "term_label": "box C/D sno(s)RNA 3'-end processing"
}